mitochondrial fragmentation involved in apoptotic process [GO:0043653] (biological process) Note: Although most of the processes described under 'apoptotic mitochondrial changes' take place during the signaling phase of apoptosis, 'mitochondrial fragmentation involved in apoptotic process' cannot be confidently placed there. It is still controversial whether this process is involved in the signaling phase of apoptosis or not, so it was placed under the more generic 'apoptotic mitochondrial changes' parent rather than linked to the signaling or the execution phase until further research clarifies the matter. References: PMID:12867994 Sources: GOC:mtg_apoptosis, GOC:rk Also known as: mitochondrial fragmentation involved in apoptosis, mitochondrial fission during apoptosis Definition: The change in the morphology of the mitochondria in an apoptotic cell from a highly branched network to a fragmented vesicular form. Relationships: is a type of apoptotic mitochondrial changes [GO:0008637]